{
  "term_label": "actin cytoskeleton",
  "gene": "UniProtKB:Q9C0H9",
  "gene_symbol": "SRCIN1",
  "term_id": "GO:0015629",
  "gene_name": "SRC kinase signaling inhibitor 1"
}